{
  "gene_symbol": "PCDH10",
  "gene_name": "Protocadherin-10",
  "term_label": "cell adhesion",
  "gene": "UniProtKB:Q9P2E7",
  "term_id": "GO:0007155"
}